xylene catabolic process [GO:0042184] (biological process) Subtypes: m-xylene catabolic process [GO:0042185], o-xylene catabolic process [GO:0042186], p-xylene catabolic process [GO:0042187] Also known as: xylene breakdown, xylene catabolism, xylene degradation Sources: GOC:go_curators Definition: The chemical reactions and pathways resulting in the breakdown of xylene, a mixture of three colorless, aromatic hydrocarbon liquids, ortho-, meta- and para-xylene. Relationships: is a type of xenobiotic catabolic process [GO:0042178]; is_a GO:0042537; is a type of hydrocarbon catabolic process [GO:0120253]